starch binding [GO:2001070] (molecular function) Sources: GOC:mengo_curators Also known as: amidon binding, amylum binding Relationships: is a type of GO:0030247 Definition: Binding to starch.